{
  "gene_symbol": "S100A10",
  "gene": "UniProtKB:P60903",
  "term_id": "GO:0048306",
  "gene_name": "Protein S100-A10",
  "term_label": "calcium-dependent protein binding"
}